{
  "gene": "UniProtKB:Q6ZVX9",
  "term_id": "GO:0038023",
  "gene_name": "Membrane progestin receptor epsilon",
  "gene_symbol": "PAQR9",
  "term_label": "signaling receptor activity"
}